{
  "gene": "UniProtKB:O00548",
  "term_id": "GO:0005112",
  "term_label": "Notch binding",
  "gene_name": "Delta-like protein 1",
  "gene_symbol": "DLL1"
}